mitotic contractile ring actin filament bundle assembly [GO:1903477] (biological process) Definition: Any actin filament bundle assembly that is involved in mitotic actomyosin contractile ring assembly. Sources: GOC:TermGenie, GOC:mtg_cell_cycle, GOC:vw, GO_REF:0000060 Relationships: is a type of actomyosin contractile ring actin filament bundle assembly [GO:0071519]; is a type of mitotic actomyosin contractile ring assembly actin filament organization [GO:1903479] Also known as: actin filament bundle assembly involved in mitotic actomyosin contractile ring assembly